response to methyl methanesulfonate [GO:0072702] (biological process) Definition: Any process that results in a change in state or activity of a cell or an organism (in terms of movement, secretion, enzyme production, gene expression, etc.) as a result of a methyl methanesulfonate (MMS) stimulus. Sources: GOC:mah Also known as: response to MMS Relationships: is_a response to oxygen-containing compound [GO:1901700] Subtypes: cellular response to methyl methanesulfonate [GO:0072703]